regulation of toll-like receptor 3 signaling pathway [GO:0034139] (biological process) References: PMID:16551253, PMID:17328678 Sources: GOC:add Also known as: regulation of TLR3 signaling pathway, regulation of toll-like receptor 3 signalling pathway Relationships: is a type of regulation of cytoplasmic pattern recognition receptor signaling pathway [GO:0039531]; regulates toll-like receptor 3 signaling pathway [GO:0034138] Definition: Any process that modulates the frequency, rate, or extent of toll-like receptor 3 signaling pathway. Subtypes: negative regulation of toll-like receptor 3 signaling pathway [GO:0034140], GO:0034141